{
  "term_label": "zinc ion transmembrane transporter activity",
  "gene_name": "Proton-coupled zinc antiporter SLC30A5",
  "term_id": "GO:0005385",
  "gene": "UniProtKB:Q8TAD4",
  "gene_symbol": "SLC30A5"
}